{
  "gene": "UniProtKB:Q9NZN4",
  "term_id": "GO:0005769",
  "gene_symbol": "EHD2",
  "term_label": "early endosome",
  "gene_name": "EH domain-containing protein 2"
}